response to UV-A [GO:0070141] (biological process) Subtypes: cellular response to UV-A [GO:0071492] Relationships: is_a response to UV [GO:0009411] Also known as: response to UV-A light stimulus, response to UV-A radiation stimulus, response to UVA light stimulus, response to UVA radiation stimulus Sources: GOC:BHF, GOC:mah Definition: Any process that results in a change in state or activity of a cell or an organism (in terms of movement, secretion, enzyme production, gene expression, etc.) as a result of a UV-A radiation stimulus. UV-A radiation (UV-A light) spans the wavelengths 315 to 400 nm.